{
  "gene": "UniProtKB:Q9UHD8",
  "term_label": "GTPase activity",
  "gene_symbol": "SEPTIN9",
  "term_id": "GO:0003924",
  "gene_name": "Septin-9"
}